{
  "gene_name": "Metalloprotease TIKI2",
  "gene": "UniProtKB:A6NFA1",
  "gene_symbol": "TRABD2B",
  "term_label": "plasma membrane",
  "term_id": "GO:0005886"
}